{
  "gene": "UniProtKB:A0FGR8",
  "gene_name": "Extended synaptotagmin-2",
  "term_id": "GO:0031210",
  "gene_symbol": "ESYT2",
  "term_label": "phosphatidylcholine binding"
}